{
  "gene": "UniProtKB:Q2M238",
  "term_id": "UNKNOWN:0003",
  "gene_name": "Putative RRN3-like protein RRN3P1",
  "term_label": "Unknown cellular component",
  "gene_symbol": "RRN3P1"
}